{
  "gene": "UniProtKB:P18627",
  "term_id": "GO:0007166",
  "gene_name": "Lymphocyte activation gene 3 protein",
  "term_label": "cell surface receptor signaling pathway",
  "gene_symbol": "LAG3"
}